{
  "gene_symbol": "FANCI",
  "gene": "UniProtKB:Q9NVI1",
  "term_label": "DNA polymerase binding",
  "gene_name": "Fanconi anemia group I protein",
  "term_id": "GO:0070182"
}